{
  "term_label": "keratin filament",
  "term_id": "GO:0045095",
  "gene": "UniProtKB:Q3SY84",
  "gene_name": "Keratin, type II cytoskeletal 71",
  "gene_symbol": "KRT71"
}